positive regulation of postsynaptic membrane organization [GO:1901628] (biological process) Subtypes: GO:1904719 Also known as: positive regulation of post-synaptic membrane organization, positive regulation of postsynaptic membrane organisation, up regulation of postsynaptic membrane organisation, up regulation of postsynaptic membrane organization, up-regulation of postsynaptic membrane organisation, up-regulation of postsynaptic membrane organization, upregulation of postsynaptic membrane organisation, upregulation of postsynaptic membrane organization, activation of postsynaptic membrane organisation, activation of postsynaptic membrane organization Relationships: is a type of positive regulation of cellular component organization [GO:0051130]; is a type of regulation of postsynaptic membrane organization [GO:1901626]; positively regulates GO:0001941 Definition: Any process that activates or increases the frequency, rate or extent of postsynaptic membrane organization. References: PMID:22426000 Sources: GOC:TermGenie